negative regulation of cytokinesis, site selection [GO:2000075] (BP) Relationships: is a type of negative regulation of cytokinesis [GO:0032466]; is a type of regulation of cytokinesis, site selection [GO:2000073]; negatively regulates cytokinesis, division site positioning [GO:0007105] Sources: GOC:mtg_cell_cycle, GOC:obol Definition: Any process that stops, prevents, or reduces the frequency, rate or extent of site selection that occurs as part of cytokinesis. Also known as: negative regulation of site selection involved in cell cycle cytokinesis